{
  "gene": "UniProtKB:P0CI01",
  "gene_symbol": "SPDYE6",
  "term_label": "Unknown biological process",
  "term_id": "UNKNOWN:0002",
  "gene_name": "Speedy protein E6"
}